{
  "gene_name": "B-cell lymphoma 3 protein",
  "term_id": "GO:0033257",
  "gene_symbol": "BCL3",
  "term_label": "Bcl3/NF-kappaB2 complex",
  "gene": "UniProtKB:P20749"
}